{
  "term_label": "protein kinase activator activity",
  "gene_name": "MOB kinase activator 3B",
  "term_id": "GO:0030295",
  "gene": "UniProtKB:Q86TA1",
  "gene_symbol": "MOB3B"
}